positive regulation of humoral immune response [GO:0002922] (biological process) Also known as: up regulation of humoral immune response, up-regulation of humoral immune response, upregulation of humoral immune response, activation of humoral immune response, stimulation of humoral immune response Sources: GOC:add Definition: Any process that activates or increases the frequency, rate, or extent of a humoral immune response. Subtypes: positive regulation of antimicrobial humoral response [GO:0002760], positive regulation of humoral immune response mediated by circulating immunoglobulin [GO:0002925], positive regulation of complement activation [GO:0045917] Relationships: is a type of regulation of humoral immune response [GO:0002920]; is_a positive regulation of immune response [GO:0050778]; positively regulates humoral immune response [GO:0006959]